{
  "gene_symbol": "CABLES1",
  "gene_name": "CDK5 and ABL1 enzyme substrate 1",
  "term_label": "nervous system development",
  "gene": "UniProtKB:Q8TDN4",
  "term_id": "GO:0007399"
}